{
  "gene_name": "Very-long-chain (3R)-3-hydroxyacyl-CoA dehydratase 4",
  "term_label": "fatty acid elongation",
  "term_id": "GO:0030497",
  "gene": "UniProtKB:Q5VWC8",
  "gene_symbol": "HACD4"
}